{
  "term_label": "Unknown molecular function",
  "gene_symbol": "KRTAP19-7",
  "term_id": "UNKNOWN:0001",
  "gene": "UniProtKB:Q3SYF9",
  "gene_name": "Keratin-associated protein 19-7"
}